{
  "gene_symbol": "NRROS",
  "gene": "UniProtKB:Q86YC3",
  "gene_name": "Transforming growth factor beta activator LRRC33",
  "term_label": "inflammatory response",
  "term_id": "GO:0006954"
}